{
  "gene_name": "Serine_threonine-protein phosphatase 2A 56 kDa regulatory subunit delta isoform",
  "term_id": "GO:0005634",
  "gene": "UniProtKB:Q14738",
  "term_label": "nucleus",
  "gene_symbol": "PPP2R5D"
}